negative regulation of cellular response to alkaline pH [GO:1900068] (biological process) Definition: Any process that stops, prevents or reduces the frequency, rate or extent of cellular response to alkalinity. References: PMID:12509465, PMID:17023428 Sources: GOC:TermGenie, GOC:dgf Also known as: negative regulation of cellular response to alkalinity, down regulation of cellular response to alkaline pH, down regulation of cellular response to basic pH, down-regulation of cellular response to alkaline pH, down-regulation of cellular response to basic pH, downregulation of cellular response to alkaline pH, downregulation of cellular response to basic pH, negative regulation of cellular response to basic pH, inhibition of cellular response to alkaline pH, inhibition of cellular response to alkalinity, inhibition of cellular response to basic pH, down regulation of cellular response to alkalinity, down-regulation of cellular response to alkalinity, downregulation of cellular response to alkalinity Relationships: is a type of GO:0048523; is a type of negative regulation of response to stimulus [GO:0048585]; is a type of regulation of cellular response to alkaline pH [GO:1900067]; negatively regulates GO:0071469